{
  "term_label": "Unknown molecular function",
  "gene_name": "Ladinin-1",
  "term_id": "UNKNOWN:0001",
  "gene_symbol": "LAD1",
  "gene": "UniProtKB:O00515"
}